{
  "gene_name": "Brefeldin A-inhibited guanine nucleotide-exchange protein 2",
  "gene": "UniProtKB:Q9Y6D5",
  "term_id": "GO:0006893",
  "gene_symbol": "ARFGEF2",
  "term_label": "Golgi to plasma membrane transport"
}